ribonucleoside-diphosphate reductase activity, glutaredoxin disulfide as acceptor [GO:0036175] (molecular function) References: PMID:19176520, PMID:31266802, PMID:7476363 Sources: GOC:bf, GOC:pde Definition: Catalysis of the reaction: 2'-deoxyribonucleoside diphosphate + glutaredoxin disulfide + H2O = ribonucleoside diphosphate + glutaredoxin. Relationships: is a type of ribonucleoside-diphosphate reductase activity [GO:0061731]